{
  "gene_name": "Beta-arrestin-2",
  "gene": "UniProtKB:P32121",
  "gene_symbol": "ARRB2",
  "term_id": "GO:0050804",
  "term_label": "modulation of chemical synaptic transmission"
}